cytoplasmic cyclin-dependent protein kinase holoenzyme complex [GO:0000308] (cellular component) Definition: Cyclin-dependent protein kinase (CDK) complex found in the cytoplasm. Sources: GOC:krc Also known as: CDK holoenzyme Relationships: is a type of cyclin-dependent protein kinase holoenzyme complex [GO:0000307]; is part of cytoplasm [GO:0005737]